{
  "term_id": "GO:0042059",
  "gene": "UniProtKB:Q9C004",
  "gene_name": "Protein sprouty homolog 4",
  "term_label": "negative regulation of epidermal growth factor receptor signaling pathway",
  "gene_symbol": "SPRY4"
}